{
  "term_label": "antigen binding",
  "gene": "UniProtKB:P01742",
  "term_id": "GO:0003823",
  "gene_name": "Immunoglobulin heavy variable 1-69",
  "gene_symbol": "IGHV1-69"
}